{
  "gene_symbol": "HSPA4L",
  "term_label": "protein folding",
  "gene_name": "Heat shock 70 kDa protein 4L",
  "gene": "UniProtKB:O95757",
  "term_id": "GO:0006457"
}